{
  "gene": "UniProtKB:P19022",
  "term_id": "GO:0044331",
  "gene_name": "Cadherin-2",
  "term_label": "cell-cell adhesion mediated by cadherin",
  "gene_symbol": "CDH2"
}